{
  "gene": "UniProtKB:P0DO92",
  "term_label": "Unknown cellular component",
  "gene_symbol": "CDIPTOSP",
  "gene_name": "Putative protein T-ENOL",
  "term_id": "UNKNOWN:0003"
}